structural constituent of bone [GO:0008147] (molecular function) Definition: The action of a molecule that contributes to the structural integrity of bone. Sources: GOC:mah Relationships: is a type of structural molecule activity [GO:0005198]